{
  "term_id": "GO:0008360",
  "gene_name": "Formin-like protein 3",
  "gene": "UniProtKB:Q8IVF7",
  "gene_symbol": "FMNL3",
  "term_label": "regulation of cell shape"
}